{
  "term_label": "Unknown biological process",
  "gene": "UniProtKB:Q11130",
  "term_id": "UNKNOWN:0002",
  "gene_name": "Alpha-(1,3)-fucosyltransferase 7",
  "gene_symbol": "FUT7"
}